purine nucleoside triphosphate metabolic process [GO:0009144] (biological process) Subtypes: purine nucleoside triphosphate biosynthetic process [GO:0009145], purine nucleoside triphosphate catabolic process [GO:0009146], GO:0009205, GO:0009215 Definition: The chemical reactions and pathways involving purine nucleoside triphosphate, a compound consisting of a purine base linked to a ribose or deoxyribose sugar esterified with triphosphate on the sugar. Also known as: purine nucleoside triphosphate metabolism Relationships: is_a nucleoside triphosphate metabolic process [GO:0009141] Sources: GOC:go_curators, ISBN:0198506732